actin body [GO:0099079] (cellular component) Definition: An amorphous cytoskeletal structure consisting of aggregated actin filaments and associated proteins (including fibrin and capping protein) in which there is little or no actin filament turnover. In yeast (S. pombe and S. cerevisiae) these are found only in quiescent cells and are thought to serve as a reserve store of actin. References: PMID:16914523 Relationships: is a type of cellular anatomical structure [GO:0110165]; BFO_0000050 GO:0015629